{
  "term_label": "Unknown cellular component",
  "gene_symbol": "EPSTI1",
  "term_id": "UNKNOWN:0003",
  "gene_name": "Epithelial-stromal interaction protein 1",
  "gene": "UniProtKB:Q96J88"
}